{
  "gene_symbol": "GPATCH3",
  "gene_name": "G patch domain-containing protein 3",
  "gene": "UniProtKB:Q96I76",
  "term_id": "GO:0032480",
  "term_label": "negative regulation of type I interferon production"
}